negative regulation of hypoxanthine transport [GO:0035347] (biological process) Also known as: negative regulation of 6-hydroxypurine transport Relationships: is a type of GO:0032240; is_a GO:0035345; negatively regulates hypoxanthine transport [GO:0035344] Definition: Any process that stops, prevents, or reduces the frequency, rate or extent of the directed movement of hypoxanthine into, out of or within a cell, or between cells, by means of some agent such as a transporter or pore. Sources: GOC:bf